{
  "term_label": "cytoplasm",
  "gene": "UniProtKB:Q8WTU0",
  "gene_symbol": "DDI1",
  "term_id": "GO:0005737",
  "gene_name": "Protein DDI1 homolog 1"
}